{
  "gene_name": "Transmembrane protein 132D",
  "term_id": "UNKNOWN:0001",
  "term_label": "Unknown molecular function",
  "gene": "UniProtKB:Q14C87",
  "gene_symbol": "TMEM132D"
}